{
  "gene_symbol": "SP6",
  "gene": "UniProtKB:Q3SY56",
  "gene_name": "Transcription factor Sp6",
  "term_label": "regulation of transcription by RNA polymerase II",
  "term_id": "GO:0006357"
}